{
  "gene": "UniProtKB:O00506",
  "term_id": "GO:0035556",
  "gene_symbol": "STK25",
  "term_label": "intracellular signal transduction",
  "gene_name": "Serine_threonine-protein kinase 25"
}